mitotic nuclear bridge organization [GO:0140515] (biological process) References: PMID:32848252 Relationships: is a type of mitotic nuclear membrane organization [GO:0101024] Definition: A mitotic cell cycle process which results in the assembly, arrangement, or disassembly of the mitotic nuclear bridge during closed mitosis.